{
  "gene_name": "High affinity cAMP-specific and IBMX-insensitive 3',5'-cyclic phosphodiesterase 8A",
  "term_id": "GO:0071364",
  "gene_symbol": "PDE8A",
  "term_label": "cellular response to epidermal growth factor stimulus",
  "gene": "UniProtKB:O60658"
}